metaxylem development [GO:0090058] (biological process) Sources: GOC:dph, GOC:sdb_2009, GOC:tb Relationships: is a type of xylem development [GO:0010089] Regulation: RO_0002211 by regulation of metaxylem development [GO:0090060] Definition: The process whose specific outcome is the progression of the metaxylem over time, from its formation to the mature structure. The metaxylem is the part of the primary xylem that differentiates after the protoxylem and before the secondary xylem, if any of the latter is formed.